{
  "gene_name": "ER degradation-enhancing alpha-mannosidase-like protein 2",
  "term_label": "endoplasmic reticulum unfolded protein response",
  "term_id": "GO:0030968",
  "gene_symbol": "EDEM2",
  "gene": "UniProtKB:Q9BV94"
}